plasmid copy number maintenance [GO:0060908] (BP) Sources: GOC:dph, GOC:tb Relationships: is a type of GO:0006276 Definition: The maintenance of the number of copies of extrachromosomal plasmid DNA.